{
  "gene_name": "Transcription termination factor 2",
  "term_id": "GO:0008094",
  "gene_symbol": "TTF2",
  "term_label": "ATP-dependent activity, acting on DNA",
  "gene": "UniProtKB:Q9UNY4"
}